{
  "gene_symbol": "LOXL4",
  "term_id": "GO:0005615",
  "term_label": "extracellular space",
  "gene": "UniProtKB:Q96JB6",
  "gene_name": "Lysyl oxidase homolog 4"
}